ABC-type cysteine transporter activity [GO:0033230] (MF) References: PMID:25837721, PMID:32144203 Sources: RHEA:29783 Also known as: ATP-dependent cysteine transporter activity, cysteine-transporting ATPase activity, ATPase-coupled cysteine transmembrane transporter activity, ATPase-coupled cysteine transporter activity, cysteine exporter, cysteine-exporting ATPase activity Definition: Enables the transfer of a solute or solutes from one side of a membrane to the other according to the reaction: ATP + H2O + L-cysteine(in) = ADP + H+ + L-cysteine(out) + phosphate. Relationships: is a type of ABC-type amino acid transporter activity [GO:0015424]; is a type of GO:0033229; is a type of ATPase-coupled carboxylic acid transmembrane transporter activity [GO:0033284]